{
  "term_id": "GO:0047086",
  "term_label": "ketosteroid monooxygenase activity",
  "gene_name": "Aldo-keto reductase family 1 member C4",
  "gene_symbol": "AKR1C4",
  "gene": "UniProtKB:P17516"
}